regulation of nucleoside metabolic process [GO:0009118] (biological process) Definition: Any process that modulates the frequency, rate or extent of the chemical reactions and pathways involving nucleosides. Relationships: is_a regulation of nucleobase-containing compound metabolic process [GO:0019219]; is a type of regulation of small molecule metabolic process [GO:0062012]; regulates GO:0009116 Sources: GOC:go_curators Subtypes: GO:0045978, positive regulation of nucleoside metabolic process [GO:0045979] Also known as: regulation of nucleoside metabolism